{
  "gene_name": "Testis, prostate and placenta-expressed protein",
  "gene_symbol": "SPMIP8",
  "gene": "UniProtKB:Q6URK8",
  "term_label": "Unknown biological process",
  "term_id": "UNKNOWN:0002"
}